intracellular glutamate homeostasis [GO:0090461] (biological process) Sources: GOC:tb Definition: A homeostatic process involved in the maintenance of a steady state level of glutamate within a cell. Relationships: is a type of intracellular amino acid homeostasis [GO:0080144] Also known as: cellular glutamate homeostasis, glutamate homeostasis